lysophosphatidic acid binding [GO:0035727] (molecular function) Sources: GOC:curators Definition: Binding to lysophosphatidic acid (LPA), a phospholipid derivative that acts as a potent mitogen due to its activation of high-affinity G protein-coupled receptors. Relationships: is a type of phospholipid binding [GO:0005543]; is a type of GO:0043168; is a type of carbohydrate derivative binding [GO:0097367] Also known as: LPA binding